{
  "term_id": "GO:0042102",
  "gene": "UniProtKB:P33681",
  "term_label": "positive regulation of T cell proliferation",
  "gene_symbol": "CD80",
  "gene_name": "T-lymphocyte activation antigen CD80"
}